{
  "gene_name": "Putative transcript Y 10 protein",
  "gene_symbol": "TTTY10",
  "gene": "UniProtKB:Q9BZA0",
  "term_label": "Unknown biological process",
  "term_id": "UNKNOWN:0002"
}